{
  "gene": "UniProtKB:P09228",
  "term_label": "extracellular space",
  "gene_name": "Cystatin-SA",
  "gene_symbol": "CST2",
  "term_id": "GO:0005615"
}